amine metabolic process [GO:0009308] (biological process) Regulation: regulated by regulation of amine metabolic process [GO:0033238]; negatively regulated by GO:0033239; positively regulated by GO:0033240 Sources: GOC:jl, ISBN:0198506732 Also known as: amine metabolism, cellular amine metabolic process Definition: The chemical reactions and pathways involving any organic compound that is weakly basic in character and contains an amino or a substituted amino group. Amines are called primary, secondary, or tertiary according to whether one, two, or three carbon atoms are attached to the nitrogen atom. Subtypes: biogenic amine metabolic process [GO:0006576], ethanolamine metabolic process [GO:0006580], amine biosynthetic process [GO:0009309], amine catabolic process [GO:0009310], cytokinin metabolic process [GO:0009690], methylamine metabolic process [GO:0030416], GO:2001129, methane biosynthetic process from trimethylamine [GO:2001130] Relationships: is a type of metabolic process [GO:0008152]